nodulation [GO:0009877] (biological process) Definition: The formation of nitrogen-fixing root nodules on plant roots. References: PMID:21856632, PMID:33317178 Also known as: nodule development, nodule formation, nodule morphogenesis Relationships: is a type of anatomical structure formation involved in morphogenesis [GO:0048646]